{
  "term_label": "protein folding",
  "gene_symbol": "PFDN4",
  "gene": "UniProtKB:Q9NQP4",
  "gene_name": "Prefoldin subunit 4",
  "term_id": "GO:0006457"
}